{
  "gene_symbol": "NPM1",
  "gene_name": "Nucleophosmin",
  "gene": "UniProtKB:P06748",
  "term_id": "GO:0010824",
  "term_label": "regulation of centrosome duplication"
}